{
  "gene": "UniProtKB:P82914",
  "term_id": "GO:0005763",
  "gene_name": "Small ribosomal subunit protein uS15m",
  "gene_symbol": "MRPS15",
  "term_label": "mitochondrial small ribosomal subunit"
}